{
  "term_id": "GO:0005634",
  "gene_name": "Probable ATP-dependent RNA helicase DDX10",
  "gene": "UniProtKB:Q13206",
  "term_label": "nucleus",
  "gene_symbol": "DDX10"
}